{
  "gene_symbol": "SNX12",
  "gene_name": "Sorting nexin-12",
  "term_id": "GO:0032456",
  "gene": "UniProtKB:Q9UMY4",
  "term_label": "endocytic recycling"
}